{
  "term_id": "UNKNOWN:0002",
  "gene": "UniProtKB:Q0VAF6",
  "gene_symbol": "SYCN",
  "gene_name": "Syncollin",
  "term_label": "Unknown biological process"
}